{
  "gene": "UniProtKB:P07954",
  "gene_name": "Fumarate hydratase, mitochondrial",
  "term_label": "mitochondrion",
  "gene_symbol": "FH",
  "term_id": "GO:0005739"
}